regulation of Fc receptor mediated stimulatory signaling pathway [GO:0060368] (biological process) Definition: Any process that modulates the rate, frequency or extent of the Fc receptor mediated stimulatory signaling pathway.. Sources: GOC:dph, GOC:tb Subtypes: GO:0060369, regulation of Fc-gamma receptor signaling pathway involved in phagocytosis [GO:1905449] Also known as: regulation of Fc receptor mediated stimulatory signalling pathway Relationships: is a type of GO:0009966; is a type of regulation of immune response [GO:0050776]; regulates Fc receptor mediated stimulatory signaling pathway [GO:0002431]